negative regulation of cell-cell adhesion [GO:0022408] (BP) Sources: GOC:isa_complete Relationships: is a type of negative regulation of cell adhesion [GO:0007162]; is a type of GO:0022407; negatively regulates GO:0098609 Also known as: down regulation of cell-cell adhesion, down-regulation of cell-cell adhesion, downregulation of cell-cell adhesion, inhibition of cell-cell adhesion Subtypes: negative regulation of cell-glial cell adhesion involved in cerebral cortex lamination [GO:0021821], negative regulation of cell-cell adhesion mediated by integrin [GO:0033633], GO:0034111, negative regulation of heterotypic cell-cell adhesion [GO:0034115], GO:0046588, negative regulation of calcium-independent cell-cell adhesion [GO:0051042], delamination [GO:0060232], negative regulation of flocculation [GO:0060257], negative regulation of leukocyte cell-cell adhesion [GO:1903038], negative regulation of homophilic cell adhesion [GO:1903386], negative regulation of epithelial cell-cell adhesion involved in epithelium migration [GO:1903682], negative regulation of cell-cell adhesion mediated by cadherin [GO:2000048] Definition: Any process that stops, prevents or reduces the rate or extent of cell adhesion to another cell.